{
  "gene_symbol": "GDF10",
  "term_label": "cytokine activity",
  "gene": "UniProtKB:P55107",
  "term_id": "GO:0005125",
  "gene_name": "Growth_differentiation factor 10"
}